endo-alpha-bergamotene synthase activity [GO:0102060] (molecular function) Definition: Catalysis of the reaction: 2-cis,6-cis-farnesyl diphosphate = (-)-endo-alpha-bergamotene + diphosphoric acid. Relationships: is a type of carbon-oxygen lyase activity, acting on phosphates [GO:0016838] Also known as: endo-alpha-bergamontene synthase activity Sources: GOC:pz, RHEA:30471